transcription factor TFIIF complex [GO:0005674] (cellular component) References: PMID:7597077 Sources: GOC:jl Definition: A general transcription initiation factor which in humans consists of a heterodimer of an alpha and a beta subunit. Helps recruit RNA polymerase II to the initiation complex and promotes translation elongation. Relationships: is a type of RNA polymerase II transcription regulator complex [GO:0090575]; is part of RNA polymerase II, holoenzyme [GO:0016591]